{
  "gene": "UniProtKB:Q8IXZ3",
  "gene_name": "Transcription factor Sp8",
  "gene_symbol": "SP8",
  "term_label": "DNA-binding transcription factor activity, RNA polymerase II-specific",
  "term_id": "GO:0000981"
}